{
  "term_label": "guanine deaminase activity",
  "gene_symbol": "GDA",
  "gene_name": "Guanine deaminase",
  "gene": "UniProtKB:Q9Y2T3",
  "term_id": "GO:0008892"
}